{
  "term_label": "Unknown cellular component",
  "gene_symbol": "LENEP",
  "gene_name": "Lens epithelial cell protein LEP503",
  "gene": "UniProtKB:Q9Y5L5",
  "term_id": "UNKNOWN:0003"
}